{
  "term_label": "calcium-mediated signaling",
  "gene": "UniProtKB:P32302",
  "gene_symbol": "CXCR5",
  "gene_name": "C-X-C chemokine receptor type 5",
  "term_id": "GO:0019722"
}